{
  "gene_name": "Probable protein phosphatase 1N",
  "gene_symbol": "PPM1N",
  "term_label": "regulation of canonical NF-kappaB signal transduction",
  "term_id": "GO:0043122",
  "gene": "UniProtKB:Q8N819"
}